{
  "gene": "UniProtKB:Q9Y6K5",
  "gene_symbol": "OAS3",
  "term_id": "GO:0060337",
  "gene_name": "2'-5'-oligoadenylate synthase 3",
  "term_label": "type I interferon-mediated signaling pathway"
}